phagocytosis, recognition [GO:0006910] (biological process) Sources: GOC:curators, ISBN:0781735149 Also known as: recognition of phagocytosed substance by phagocytic cell Note: Note that cell surface molecules involved in the direct binding of bacteria may be also annotated to the molecular function term 'bacterial cell surface binding ; GO:0051635'. Note that cell surface molecules involved in the direct binding to opsonins such as complement components or antibodies may be also annotated to the term 'opsonin binding ; GO:0001846'. Subtypes: recognition of apoptotic cell [GO:0043654] Relationships: is a type of cell recognition [GO:0008037]; is part of GO:0006909; BFO_0000051 cargo receptor activity [GO:0038024] Regulation: positively regulated by opsonization [GO:0008228] Definition: The initial step in phagocytosis involving adhesion to bacteria, immune complexes and other particulate matter, or an apoptotic cell and based on recognition of factors such as bacterial cell wall components, opsonins like complement and antibody or protein receptors and lipids like phosphatidyl serine, and leading to intracellular signaling in the phagocytosing cell.